{
  "gene_symbol": "SLC9C2",
  "term_label": "sodium:proton antiporter activity",
  "gene_name": "Sodium_hydrogen exchanger 11",
  "gene": "UniProtKB:Q5TAH2",
  "term_id": "GO:0015385"
}